{
  "gene_name": "Golgi-associated RAB2 interactor protein 2",
  "term_label": "Unknown molecular function",
  "gene_symbol": "GARIN2",
  "gene": "UniProtKB:Q8N9W8",
  "term_id": "UNKNOWN:0001"
}